{
  "gene_name": "Probable ubiquitin carboxyl-terminal hydrolase MINDY-4",
  "gene_symbol": "MINDY4",
  "term_label": "Unknown biological process",
  "gene": "UniProtKB:Q4G0A6",
  "term_id": "UNKNOWN:0002"
}